{
  "term_id": "GO:0030215",
  "gene_name": "Semaphorin-3C",
  "term_label": "semaphorin receptor binding",
  "gene_symbol": "SEMA3C",
  "gene": "UniProtKB:Q99985"
}